{
  "term_label": "Unknown molecular function",
  "term_id": "UNKNOWN:0001",
  "gene_name": "Craniofacial development protein 1",
  "gene_symbol": "CFDP1",
  "gene": "UniProtKB:Q9UEE9"
}